negative regulation of meiotic cell cycle [GO:0051447] (biological process) Also known as: down regulation of progression through meiotic cell cycle, down-regulation of progression through meiotic cell cycle, downregulation of progression through meiotic cell cycle, negative regulation of meiotic cell cycle progression, negative regulation of progression through meiotic cell cycle, inhibition of progression through meiotic cell cycle Sources: GOC:ai, GOC:dph, GOC:tb Definition: Any process that stops, prevents or reduces the rate or extent of progression through the meiotic cell cycle. Subtypes: GO:0043942, GO:0045835, negative regulation of meiotic cell cycle phase transition [GO:1901994], GO:1904145, negative regulation of initiation of premeiotic DNA replication [GO:1904513] Relationships: is a type of negative regulation of cell cycle [GO:0045786]; is a type of regulation of meiotic cell cycle [GO:0051445]; is a type of negative regulation of reproductive process [GO:2000242]; negatively regulates meiotic cell cycle [GO:0051321]